{
  "gene": "UniProtKB:P23527",
  "gene_name": "Histone H2B type 1-O",
  "gene_symbol": "H2BC17",
  "term_id": "GO:0019731",
  "term_label": "antibacterial humoral response"
}